{
  "term_label": "Unknown biological process",
  "gene_name": "Putative uncharacterized protein encoded by LINC00167",
  "term_id": "UNKNOWN:0002",
  "gene_symbol": "PRDM10-DT",
  "gene": "UniProtKB:Q96N53"
}